D-xylose catabolic process to ethanol [GO:0044577] (biological process) Also known as: D-xylose fermentation, xylose catabolism to ethanol Relationships: is a type of GO:0006067; is a type of GO:0006113; is a type of D-xylose catabolic process [GO:0042843] Regulation: RO_0002211 by regulation of xylose catabolic process to ethanol [GO:1900515]; RO_0002212 by negative regulation of xylose catabolic process to ethanol [GO:1900516]; positively regulated by positive regulation of xylose catabolic process to ethanol [GO:1900517] Definition: The anaerobic chemical reactions and pathways resulting in the breakdown of xylose, an aldopentose, into ethanol. References: PMID:26927067 Sources: GOC:mengo_curators, GOC:tt